{
  "term_label": "ubiquitin-like ligase-substrate adaptor activity",
  "term_id": "GO:1990756",
  "gene_symbol": "KBTBD3",
  "gene_name": "Kelch repeat and BTB domain-containing protein 3",
  "gene": "UniProtKB:Q8NAB2"
}